{
  "term_label": "transcription initiation at RNA polymerase II promoter",
  "gene_name": "Transcription initiation factor TFIID subunit 10",
  "gene": "UniProtKB:Q12962",
  "gene_symbol": "TAF10",
  "term_id": "GO:0006367"
}